{
  "gene": "UniProtKB:Q06830",
  "term_label": "thioredoxin peroxidase activity",
  "gene_symbol": "PRDX1",
  "term_id": "GO:0008379",
  "gene_name": "Peroxiredoxin-1"
}